post-embryonic ectodermal digestive tract development [GO:0048612] (biological process) Definition: The process, occurring during the post-embryonic phase, whose specific outcome is the progression of the ectodermal gut over time, from its formation to the mature structure. Sources: GOC:jid, GOC:rc Also known as: post-embryonic ectodermal gut development Relationships: is a type of ectodermal digestive tract development [GO:0007439]